{
  "term_label": "Cul4-RING E3 ubiquitin ligase complex",
  "gene_name": "WD and tetratricopeptide repeats protein 1",
  "gene": "UniProtKB:Q8N5D0",
  "gene_symbol": "WDTC1",
  "term_id": "GO:0080008"
}